{
  "gene": "UniProtKB:Q9NXN4",
  "gene_name": "Ganglioside-induced differentiation-associated protein 2",
  "gene_symbol": "GDAP2",
  "term_id": "UNKNOWN:0002",
  "term_label": "Unknown biological process"
}